{
  "gene_symbol": "CXCR6",
  "gene_name": "C-X-C chemokine receptor type 6",
  "gene": "UniProtKB:O00574",
  "term_id": "GO:0016493",
  "term_label": "C-C chemokine receptor activity"
}